{
  "gene_name": "Isocitrate dehydrogenase [NAD] subunit gamma, mitochondrial",
  "gene": "UniProtKB:P51553",
  "term_label": "mitochondrion",
  "gene_symbol": "IDH3G",
  "term_id": "GO:0005739"
}